{
  "gene_name": "Olfactory receptor 1N2",
  "term_label": "plasma membrane",
  "gene": "UniProtKB:Q8NGR9",
  "term_id": "GO:0005886",
  "gene_symbol": "OR1N2"
}